{
  "term_id": "UNKNOWN:0002",
  "term_label": "Unknown biological process",
  "gene_symbol": "RASSF7",
  "gene": "UniProtKB:Q02833",
  "gene_name": "Ras association domain-containing protein 7"
}